pericyte cell migration [GO:1905351] (biological process) Relationships: is a type of cell migration [GO:0016477] Definition: The orderly movement of a pericyte cell from one site to another. References: PMID:26268439 Sources: GOC:BHF, GOC:BHF_miRNA, GOC:TermGenie, GOC:rph, GO_REF:0000091